glucan metabolic process [GO:0044042] (biological process) Sources: GOC:jl Also known as: glucan metabolism Subtypes: glycogen metabolic process [GO:0005977], starch metabolic process [GO:0005982], GO:0009250, glucan catabolic process [GO:0009251], xyloglucan metabolic process [GO:0010411], alpha-glucan metabolic process [GO:0030978], GO:0051273, glucosylglycerol metabolic process [GO:0051472], pullulan metabolic process [GO:0051676], cellodextrin metabolic process [GO:2000889], cyclodextrin metabolic process [GO:2000900] Relationships: is a type of GO:0005976 Definition: The chemical reactions and pathways involving glucans, polysaccharides consisting only of glucose residues.